{
  "term_label": "cardiolipin acyl-chain remodeling",
  "term_id": "GO:0035965",
  "gene_symbol": "TAFAZZIN",
  "gene_name": "Tafazzin",
  "gene": "UniProtKB:Q16635"
}